{
  "gene": "UniProtKB:Q9HC24",
  "gene_symbol": "TMBIM4",
  "term_label": "endoplasmic reticulum unfolded protein response",
  "term_id": "GO:0030968",
  "gene_name": "Protein lifeguard 4"
}